{
  "gene": "UniProtKB:Q86UL8",
  "gene_symbol": "MAGI2",
  "term_label": "cytoplasm",
  "term_id": "GO:0005737",
  "gene_name": "Membrane-associated guanylate kinase, WW and PDZ domain-containing protein 2"
}